{
  "gene": "UniProtKB:Q15413",
  "gene_symbol": "RYR3",
  "term_label": "sarcolemma",
  "term_id": "GO:0042383",
  "gene_name": "Ryanodine receptor 3"
}